reproductive process [GO:0022414] (biological process) Regulation: regulated by regulation of reproductive process [GO:2000241]; negatively regulated by negative regulation of reproductive process [GO:2000242]; positively regulated by GO:2000243 Definition: A biological process that directly contributes to the process of producing new individuals by one or two organisms. The new individuals inherit some proportion of their genetic material from the parent or parents. Relationships: is a type of biological_process [GO:0008150] Subtypes: GO:0003006, acrosome reaction [GO:0007340], embryo implantation [GO:0007566], fertilization [GO:0009566], pollination [GO:0009856], sexual reproduction [GO:0019953], GO:0019954, reproductive process in single-celled organism [GO:0022413], ovulation cycle process [GO:0022602], mating plug formation [GO:0042628], multi-organism reproductive process [GO:0044703], multicellular organismal reproductive process [GO:0048609], meiotic cell cycle [GO:0051321], positive regulation of flagellated sperm motility involved in capacitation [GO:0060474], premature acrosome loss [GO:0061948], spore dispersal [GO:0075325], GO:0097722, GO:0110134, meiotic cell cycle process [GO:1903046], parasexual reproduction with cellular fusion [GO:1990277] Also known as: single organism reproductive process Sources: GOC:dph, GOC:isa_complete